GDP-4-dehydro-D-rhamnose reductase activity [GO:0042356] (molecular function) Sources: EC:1.1.1.187 Definition: Catalysis of the reaction: GDP-6-deoxy-D-mannose + NAD(P)+ = GDP-4-dehydro-6-deoxy-D-mannose + NAD(P)H + H+. In the reverse reaction, a mixture of GDP-D-rhamnose and its C-4 epimer is formed. Also known as: GDP-4-keto-6-deoxy-D-mannose reductase activity, GDP-4-keto-D-rhamnose reductase activity, GDP-6-deoxy-D-mannose:NAD(P)+ 4-oxidoreductase activity, guanosine diphosphate-4-keto-D-rhamnose reductase activity Relationships: is_a oxidoreductase activity, acting on the CH-OH group of donors, NAD or NADP as acceptor [GO:0016616]